{
  "gene": "UniProtKB:O95347",
  "term_label": "condensed chromosome",
  "gene_name": "Structural maintenance of chromosomes protein 2",
  "term_id": "GO:0000793",
  "gene_symbol": "SMC2"
}